positive regulation of fibroblast growth factor receptor signaling pathway involved in neural plate anterior/posterior pattern formation [GO:2000315] (biological process) Sources: GOC:BHF Definition: Any process that activates or increases the frequency, rate or extent of fibroblast growth factor receptor signaling pathway involved in neural plate anterior/posterior pattern formation. Also known as: positive regulation of fibroblast growth factor receptor signalling pathway involved in neural plate anterior/posterior pattern formation Relationships: is a type of positive regulation of fibroblast growth factor receptor signaling pathway [GO:0045743]; is a type of positive regulation of developmental process [GO:0051094]; is_a positive regulation of multicellular organismal process [GO:0051240]; is a type of regulation of fibroblast growth factor receptor signaling pathway involved in neural plate anterior/posterior pattern formation [GO:2000313]; positively regulates fibroblast growth factor receptor signaling pathway involved in neural plate anterior/posterior pattern formation [GO:0060825]